deoxyadenosine biosynthetic process [GO:0046091] (biological process) Relationships: is a type of GO:0046090; is a type of purine deoxyribonucleoside biosynthetic process [GO:0046123] Also known as: deoxyadenosine anabolism, deoxyadenosine biosynthesis, deoxyadenosine formation, deoxyadenosine synthesis Definition: The chemical reactions and pathways resulting in the formation of deoxyadenosine, 2-deoxyribosyladenine, one of the four major nucleosides of DNA. Sources: GOC:go_curators